{
  "gene": "UniProtKB:A0A3B3IU63",
  "gene_symbol": "H2AL3",
  "term_id": "GO:0000786",
  "term_label": "nucleosome",
  "gene_name": "Histone H2A-like 3"
}